cellular response to nitric oxide [GO:0071732] (biological process) Relationships: is a type of response to nitric oxide [GO:0071731]; is a type of cellular response to oxygen-containing compound [GO:1901701]; is a type of GO:1902170 Sources: GOC:mah, GOC:yaf Definition: Any process that results in a change in state or activity of a cell (in terms of movement, secretion, enzyme production, gene expression, etc.) as a result of a nitric oxide stimulus.